symbiont-mediated detoxification of host-generated reactive oxygen species [GO:0141082] (biological process) References: PMID:19684141, PMID:27825304, PMID:28288207 Definition: A process in which a symbiont interferes with, inhibits or disrupts the host reactive oxygen species (ROS)-mediated innate immune response by directly degrading host ROS. The host is defined as the larger of the organisms involved in a symbiotic interaction. Relationships: is a type of symbiont defense to host-produced reactive oxygen species [GO:0052164]